{
  "gene_name": "T-box transcription factor TBX10",
  "term_label": "nucleus",
  "term_id": "GO:0005634",
  "gene_symbol": "TBX10",
  "gene": "UniProtKB:O75333"
}